{
  "gene": "UniProtKB:Q9H0R6",
  "term_id": "GO:0032543",
  "gene_symbol": "QRSL1",
  "gene_name": "Glutamyl-tRNA(Gln) amidotransferase subunit A, mitochondrial",
  "term_label": "mitochondrial translation"
}